{
  "term_label": "3',5'-cyclic-AMP phosphodiesterase activity",
  "gene_symbol": "PDE6A",
  "gene": "UniProtKB:P16499",
  "term_id": "GO:0004115",
  "gene_name": "Rod cGMP-specific 3',5'-cyclic phosphodiesterase subunit alpha"
}